{
  "gene_symbol": "ZNF280C",
  "gene_name": "Zinc finger protein 280C",
  "term_id": "GO:0006355",
  "gene": "UniProtKB:Q8ND82",
  "term_label": "regulation of DNA-templated transcription"
}